{
  "gene_name": "Nuclear receptor subfamily 1 group I member 2",
  "gene_symbol": "NR1I2",
  "term_id": "GO:0005634",
  "gene": "UniProtKB:O75469",
  "term_label": "nucleus"
}